{
  "term_id": "GO:0016887",
  "gene_symbol": "HSP90AB1",
  "term_label": "ATP hydrolysis activity",
  "gene_name": "Heat shock protein HSP 90-beta",
  "gene": "UniProtKB:P08238"
}